S-adenosylmethionine-dependent methyltransferase activity [GO:0008757] (molecular function) Definition: Catalysis of the transfer of a methyl group from S-adenosyl-L-methionine to a substrate. Sources: GOC:mah Also known as: S-adenosyl methionine-dependent methyltransferase activity, SAM-dependent methyltransferase activity Relationships: is a type of methyltransferase activity [GO:0008168] Subtypes: GO:0000234, phosphatidyl-N-methylethanolamine N-methyltransferase activity [GO:0000773], sterol 24-C-methyltransferase activity [GO:0003838], GO:0003886, GO:0004164, methylene-fatty-acyl-phospholipid synthase activity [GO:0004481], phenylethanolamine N-methyltransferase activity [GO:0004603], phosphatidylethanolamine N-methyltransferase activity [GO:0004608], protein C-terminal S-isoprenylcysteine carboxyl O-methyltransferase activity [GO:0004671], protein-L-isoaspartate (D-aspartate) O-methyltransferase activity [GO:0004719], thioether S-methyltransferase activity [GO:0004790], GO:0004808, uroporphyrin-III C-methyltransferase activity [GO:0004851], nicotinamide N-methyltransferase activity [GO:0008112], thiopurine S-methyltransferase activity [GO:0008119], mRNA methyltransferase activity [GO:0008174], rRNA methyltransferase activity [GO:0008649], cyclopropane-fatty-acyl-phospholipid synthase activity [GO:0008825], S-adenosylmethionine-homocysteine S-methyltransferase activity [GO:0008898], nicotinate N-methyltransferase activity [GO:0008938], protein-glutamate O-methyltransferase activity [GO:0008983], site-specific DNA-methyltransferase (adenine-specific) activity [GO:0009007], polyprenyldihydroxybenzoate methyltransferase activity [GO:0010420], GO:0015667, catechol O-methyltransferase activity [GO:0016206], arginine N-methyltransferase activity [GO:0016273], GO:0016278, tRNA (guanine) methyltransferase activity [GO:0016423], tRNA (adenine) methyltransferase activity [GO:0016426], tRNA (cytidine) methyltransferase activity [GO:0016427], acetylserotonin O-methyltransferase activity [GO:0017096], GO:0017174, protein-L-histidine N-tele-methyltransferase activity [GO:0018064], protein C-terminal leucine carboxyl O-methyltransferase activity [GO:0018423], thiol S-methyltransferase activity [GO:0018708], farnesoic acid O-methyltransferase activity [GO:0019010], GO:0030697, guanidinoacetate N-methyltransferase activity [GO:0030731], methionine S-methyltransferase activity [GO:0030732], fatty acid O-methyltransferase activity [GO:0030733], polysaccharide O-methyltransferase activity [GO:0030734], carnosine N-methyltransferase activity [GO:0030735], phenol O-methyltransferase activity [GO:0030736], iodophenol O-methyltransferase activity [GO:0030737], tyramine N-methyltransferase activity [GO:0030738], GO:0030739, inositol 3-methyltransferase activity [GO:0030740], inositol 1-methyltransferase activity [GO:0030741], isoflavone 4'-O-methyltransferase activity [GO:0030746], GO:0030747, GO:0030748, loganate O-methyltransferase activity [GO:0030749], GO:0030750, licodione 2'-O-methyltransferase activity [GO:0030751], 5-hydroxyfuranocoumarin 5-O-methyltransferase activity [GO:0030752], 8-hydroxyfuranocoumarin 8-O-methyltransferase activity [GO:0030753], apigenin 4'-O-methyltransferase activity [GO:0030754], quercetin 3-O-methyltransferase activity [GO:0030755], isoorientin 3'-O-methyltransferase activity [GO:0030756], 3-methylquercitin 7-O-methyltransferase activity [GO:0030757], 3,7-dimethylquercitin 4'-O-methyltransferase activity [GO:0030758], methylquercetagetin 6-O-methyltransferase activity [GO:0030759], pyridine N-methyltransferase activity [GO:0030760], 8-hydroxyquercitin 8-O-methyltransferase activity [GO:0030761], tetrahydrocolumbamine 2-O-methyltransferase activity [GO:0030762], GO:0030763, GO:0030766, 3-hydroxyanthranilate 4-C-methyltransferase activity [GO:0030767], 16-methoxy-2,3-dihydro-3-hydroxytabersonine N-methyltransferase activity [GO:0030768], macrocin O-methyltransferase activity [GO:0030769], demethylmacrocin O-methyltransferase activity [GO:0030770], GO:0030771, tryptophan 2-C-methyltransferase activity [GO:0030772], 6-hydroxymellein O-methyltransferase activity [GO:0030773], anthranilate N-methyltransferase activity [GO:0030774], glucuronoxylan 4-O-methyltransferase activity [GO:0030775], (RS)-1-benzyl-1,2,3,4-tetrahydroisoquinoline N-methyltransferase activity [GO:0030776], (S)-scoulerine 9-O-methyltransferase activity [GO:0030777], columbamine O-methyltransferase activity [GO:0030778], GO:0030779, 12-hydroxydihydrochelirubine 12-O-methyltransferase activity [GO:0030780], 6-O-methylnorlaudanosoline 5'-O-methyltransferase activity [GO:0030781], GO:0030782, [cytochrome c]-methionine S-methyltransferase activity [GO:0030783], 3'-hydroxy-N-methyl-(S)-coclaurine 4'-O-methyltransferase activity [GO:0030784], GO:0030785, (RS)-norcoclaurine 6-O-methyltransferase activity [GO:0030786], inositol 4-methyltransferase activity [GO:0030787], precorrin-2 C20-methyltransferase activity [GO:0030788], GO:0030789, chlorophenol O-methyltransferase activity [GO:0030790], arsenite methyltransferase activity [GO:0030791], GO:0030793, (S)-coclaurine-N-methyltransferase activity [GO:0030794], GO:0030795, cycloartenol 24-C-methyltransferase activity [GO:0030796], 24-methylenesterol C-methyltransferase activity [GO:0030797], GO:0030798, myricetin 3'-O-methyltransferase activity [GO:0033799], isoflavone 7-O-methyltransferase activity [GO:0033800], vitexin 2''-O-rhamnoside 7-O-methyltransferase activity [GO:0033801], isoliquiritigenin 2'-O-methyltransferase activity [GO:0033802], kaempferol 4'-O-methyltransferase activity [GO:0033803], protein-arginine C-methyltransferase activity [GO:0035244], GO:0035797, protein-glutamine N-methyltransferase activity [GO:0036009], GO:0042409, GO:0043839, precorrin-6Y C5,15-methyltransferase (decarboxylating) activity [GO:0046025], precorrin-4 C11-methyltransferase activity [GO:0046026], magnesium protoporphyrin IX methyltransferase activity [GO:0046406], histamine N-methyltransferase activity [GO:0046539], GO:0046547, 2-methyl-6-phytyl-1,4-benzoquinone methyltransferase activity [GO:0051741], GO:0051742, GO:0052706, dimethylglycine N-methyltransferase activity [GO:0052729], sarcosine N-methyltransferase activity [GO:0052730], 3-demethylubiquinol 3-O-methyltransferase activity [GO:0061542], laricitrin 5'-O-methyltransferase activity [GO:0070448], RNA cap trimethylguanosine synthase activity [GO:0071164], N-terminal protein N-methyltransferase activity [GO:0071885], flavone 3'-O-methyltransferase activity [GO:0102822], 3,5-dichloro-THPH methyl transferase activity [GO:0106268], GO:0106363, protein-L-histidine N-pros-methyltransferase activity [GO:0106370], 3-demethylubiquinone 3-O-methyltransferase activity [GO:0120537], diphthine methyl ester synthase activity [GO:0141133], 4-vinylphenol methyltransferase activity [GO:0160304], RNA 5'-gamma-phosphate methyltransferase activity [GO:1990276]